{
  "gene": "UniProtKB:Q8WUY9",
  "gene_name": "DEP domain-containing protein 1B",
  "gene_symbol": "DEPDC1B",
  "term_id": "UNKNOWN:0001",
  "term_label": "Unknown molecular function"
}